{
  "gene_symbol": "USP24",
  "term_id": "GO:0004843",
  "gene": "UniProtKB:Q9UPU5",
  "gene_name": "Ubiquitin carboxyl-terminal hydrolase 24",
  "term_label": "cysteine-type deubiquitinase activity"
}